{
  "gene": "UniProtKB:Q9P2D3",
  "term_label": "Unknown molecular function",
  "term_id": "UNKNOWN:0001",
  "gene_symbol": "HEATR5B",
  "gene_name": "HEAT repeat-containing protein 5B"
}